ethanolaminephosphotransferase activity [GO:0004307] (MF) Definition: Catalysis of the reaction: CDP-ethanolamine + 1,2-diacylglycerol = CMP + a phosphatidylethanolamine. Also known as: CDP-ethanolamine:1,2-diacylglycerol ethanolaminephosphotransferase activity, CDPethanolamine diglyceride phosphotransferase activity, EPT, diacylglycerol ethanolaminephosphotransferase activity, phosphorylethanolamine-glyceride transferase activity Relationships: is a type of CDP-alcohol phosphatidyltransferase activity [GO:0017169] Sources: EC:2.7.8.1, RHEA:32943